{
  "gene_name": "Prolactin",
  "term_id": "GO:0031667",
  "gene": "UniProtKB:P01236",
  "gene_symbol": "PRL",
  "term_label": "response to nutrient levels"
}